voltage-gated proton channel activity [GO:0030171] (molecular function) Definition: Enables the transmembrane transfer of a proton by a voltage-gated channel. A voltage-gated channel is a channel whose open state is dependent on the voltage across the membrane in which it is embedded. References: PMID:28774948 Relationships: is a type of GO:0015252; is a type of voltage-gated monoatomic cation channel activity [GO:0022843] Also known as: voltage gated proton channel activity, voltage-dependent proton channel activity